{
  "gene": "UniProtKB:Q5NUL3",
  "gene_symbol": "FFAR4",
  "term_id": "GO:0046879",
  "term_label": "hormone secretion",
  "gene_name": "Free fatty acid receptor 4"
}